uterus development [GO:0060065] (BP) Sources: GOC:dph, GOC:ebc Relationships: is_a GO:0048513; is a type of reproductive structure development [GO:0048608] Also known as: Mullerian tract development Definition: The reproductive developmental process whose specific outcome is the progression of the uterus over time, from its formation to the mature structure.